ADP-ribose pyrophosphohydrolase activity [GO:0080041] (molecular function) Definition: Catalysis of the reaction: ADP-ribose + H2O = AMP + ribose-1-phosphate. Relationships: is a type of ADP-sugar diphosphatase activity [GO:0019144] Sources: GOC:tb